cell adhesive protein binding involved in bundle of His cell-Purkinje myocyte communication [GO:0086083] (molecular function) Relationships: is a type of GO:0086080; is part of bundle of His cell-Purkinje myocyte adhesion involved in cell communication [GO:0086073] Sources: GOC:BHF, GOC:mtg_cardiac_conduct_nov11 Definition: Binding to a protein or protein complex that results in the connection of a bundle of His cell with a Purkinje myocyte and contributes to the communication between the two cells.